{
  "gene": "UniProtKB:Q9NX38",
  "term_label": "actin monomer binding",
  "gene_symbol": "ABITRAM",
  "gene_name": "Protein Abitram",
  "term_id": "GO:0003785"
}